{
  "gene_name": "Myosin light polypeptide 6",
  "gene_symbol": "MYL6",
  "gene": "UniProtKB:P60660",
  "term_label": "Unknown biological process",
  "term_id": "UNKNOWN:0002"
}